{
  "gene_name": "Putative STAG3-like protein 2",
  "gene_symbol": "STAG3L2",
  "term_label": "Unknown biological process",
  "gene": "UniProtKB:P0CL84",
  "term_id": "UNKNOWN:0002"
}